{
  "gene_symbol": "ZFP64",
  "term_label": "transcription cis-regulatory region binding",
  "gene_name": "Zinc finger protein 64",
  "term_id": "GO:0000976",
  "gene": "UniProtKB:Q9NTW7"
}